{
  "gene": "UniProtKB:Q8NAA6",
  "term_id": "UNKNOWN:0001",
  "gene_symbol": "LINC02694",
  "term_label": "Unknown molecular function",
  "gene_name": "Putative uncharacterized protein encoded by LINC02694"
}